CTP synthase activity [GO:0003883] (molecular function) Also known as: CTP synthetase activity, UTP--ammonia ligase activity, UTP:ammonia ligase (ADP-forming), cytidine 5'-triphosphate synthetase activity, cytidine triphosphate synthetase activity, uridine triphosphate aminase activity Definition: Catalysis of the reaction: ATP + UTP + glutamine + H20= ADP + phosphate + CTP + glutamate. Relationships: is a type of GO:0016879 References: PMID:12354108 Sources: RHEA:26426